{
  "gene_symbol": "ATP8B1",
  "term_id": "GO:0005886",
  "term_label": "plasma membrane",
  "gene_name": "Phospholipid-transporting ATPase IC",
  "gene": "UniProtKB:O43520"
}